{
  "gene_name": "WW domain-binding protein 1",
  "gene_symbol": "WBP1",
  "term_label": "Unknown biological process",
  "gene": "UniProtKB:Q96G27",
  "term_id": "UNKNOWN:0002"
}